epicardium-derived cell migration to the myocardium [GO:0003346] (BP) References: PMID:18722343 Sources: GOC:dph Relationships: is a type of cell migration involved in heart development [GO:0060973] Definition: The orderly movement of a cell that have undergone an epithelial to mesenchymal transition from the epicardium into the myocardium.